protein K6-linked deubiquitination [GO:0044313] (biological process) Sources: GOC:sp Definition: A protein deubiquitination process in which a K6-linked ubiquitin chain, i.e. a polymer of ubiquitin formed by linkages between lysine residues at position 6 of the ubiquitin monomers, is removed from a protein. Relationships: is a type of GO:0016579